{
  "gene_name": "T cell receptor beta variable 12-5",
  "gene_symbol": "TRBV12-5",
  "term_label": "cell surface receptor signaling pathway",
  "gene": "UniProtKB:A0A1B0GX78",
  "term_id": "GO:0007166"
}